{
  "term_id": "GO:0000981",
  "gene_name": "Early growth response protein 4",
  "term_label": "DNA-binding transcription factor activity, RNA polymerase II-specific",
  "gene_symbol": "EGR4",
  "gene": "UniProtKB:Q05215"
}